{
  "term_id": "GO:0016324",
  "gene_name": "Aquaporin-2",
  "gene": "UniProtKB:P41181",
  "gene_symbol": "AQP2",
  "term_label": "apical plasma membrane"
}